{
  "gene_symbol": "PKD1L1",
  "gene_name": "Polycystin-1-like protein 1",
  "term_id": "GO:0050982",
  "term_label": "detection of mechanical stimulus",
  "gene": "UniProtKB:Q8TDX9"
}